{
  "gene": "UniProtKB:Q04727",
  "gene_symbol": "TLE4",
  "gene_name": "Transducin-like enhancer protein 4",
  "term_label": "transcription corepressor activity",
  "term_id": "GO:0003714"
}